{
  "term_id": "GO:0005634",
  "gene_name": "Death-associated protein kinase 1",
  "gene": "UniProtKB:P53355",
  "term_label": "nucleus",
  "gene_symbol": "DAPK1"
}